fumonisin catabolic process [GO:1900540] (biological process) Sources: GOC:TermGenie Also known as: fumonisin breakdown, fumonisin catabolism, fumonisin degradation Definition: The chemical reactions and pathways resulting in the breakdown of fumonisin. Relationships: is_a carboxylic acid catabolic process [GO:0046395]; is a type of GO:0090487